{
  "gene": "UniProtKB:Q8IZ20",
  "term_label": "Unknown cellular component",
  "gene_name": "Tissue-resident T-cell transcription regulator protein ZNF683",
  "gene_symbol": "ZNF683",
  "term_id": "UNKNOWN:0003"
}